{
  "term_label": "potassium:proton antiporter activity",
  "gene_name": "Sodium_hydrogen exchanger 9",
  "term_id": "GO:0015386",
  "gene": "UniProtKB:Q8IVB4",
  "gene_symbol": "SLC9A9"
}